regulation of smooth muscle cell chemotaxis [GO:0071671] (biological process) Definition: Any process that modulates the frequency, rate, or extent of smooth muscle cell chemotaxis. Sources: GOC:mah Relationships: is a type of regulation of smooth muscle cell migration [GO:0014910]; is a type of regulation of chemotaxis [GO:0050920]; regulates GO:0071670 Subtypes: negative regulation of smooth muscle cell chemotaxis [GO:0071672], positive regulation of smooth muscle cell chemotaxis [GO:0071673]